response to acidic pH [GO:0010447] (biological process) Definition: Any process that results in a change in state or activity of a cell or an organism (in terms of movement, secretion, enzyme production, gene expression, etc.) as a result of a pH stimulus with pH < 7. pH is a measure of the acidity or basicity of an aqueous solution. Also known as: response to acidity Note: This term should be used to annotate instances where a cell or organism is responding to a chemical that is playing the role of an acid (e.g. proton donor) and therefore lowering the pH. If instead you wish to describe a response to a specific acid as a chemical, such as the anion portion of glutamate, please annotate to the appropriate child of GO:0001101 'response to acid chemical'. Subtypes: cellular response to acidic pH [GO:0071468] Relationships: is a type of GO:0009268 Sources: GOC:go_curators, GOC:tb, Wikipedia:PH